histone H2AK9 acetyltransferase activity [GO:0044012] (molecular function) Relationships: is a type of GO:0043998 Also known as: histone H2A-K9 acetyltransferase activity, histone acetylase activity (H2A-K9 specific), histone acetyltransferase activity (H2A-K9 specific), histone lysine N-acetyltransferase activity (H2A-K9 specific) Note: Note that the residue position corresponds to the canonical human H2A2A histone (UniProtKB:Q6FI13); this residue is conserved across all eukaryotes. Corresponds to H2AK7 in yeast and in flies. Residue 1 is the first residue following removal of the initiating Methionine (Met). Note that each histone is encoded by multiple genes, and sequences may vary across different genes within an organism. References: PMID:18552846 Definition: Catalysis of the reaction: acetyl-CoA + histone H2A L-lysine (position 9) = CoA + histone H2A N6-acetyl-L-lysine (position 9).